{
  "gene": "UniProtKB:Q9BZM6",
  "term_label": "extracellular space",
  "gene_name": "UL16-binding protein 1",
  "term_id": "GO:0005615",
  "gene_symbol": "ULBP1"
}